{
  "gene": "UniProtKB:O60682",
  "term_id": "GO:0007519",
  "gene_symbol": "MSC",
  "gene_name": "Musculin",
  "term_label": "skeletal muscle tissue development"
}